vascular endothelial cell response to fluid shear stress [GO:0097699] (biological process) Relationships: is_a cellular response to fluid shear stress [GO:0071498] Also known as: blood vessel endothelial cell response to fluid shear stress References: PMID:21768538 Sources: GOC:BHF, GOC:BHF_miRNA, GOC:bc Definition: Any response to fluid shear stress in a vascular endothelial cell. Subtypes: vascular endothelial cell response to laminar fluid shear stress [GO:0097700], vascular endothelial cell response to pulsatile fluid shear stress [GO:0097705], vascular endothelial cell response to oscillatory fluid shear stress [GO:0097706]